{
  "gene_symbol": "FEZF1",
  "term_id": "GO:0003700",
  "gene": "UniProtKB:A0PJY2",
  "gene_name": "Fez family zinc finger protein 1",
  "term_label": "DNA-binding transcription factor activity"
}